ectoine catabolic process [GO:0042400] (biological process) References: PMID:11823218 Sources: GOC:jl Definition: The chemical reactions and pathways resulting in the breakdown of ectoine (1,4,5,6-tetrahydro-2-methyl-4-pyrimidinecarboxylic acid), a tetrahydropyrimidine commonly synthesized by halophilic bacteria. Relationships: is a type of monocarboxylic acid catabolic process [GO:0072329] Also known as: ectoine breakdown, ectoine catabolism, ectoine degradation